ferredoxin-thioredoxin reductase complex [GO:0030386] (cellular component) Definition: A protein complex that possesses ferredoxin-thioredoxin reductase activity. Note: Note that this term represents a location and not a function; the activity possessed by this complex is mentioned in the definition for the purpose of describing and distinguishing the complex. The function possessed by this complex is represented by the molecular function term 'ferredoxin-thioredoxin reductase activity ; GO:0103012'. Also known as: ferredoxin:thioredoxin reductase complex Relationships: is_a oxidoreductase complex [GO:1990204]; is part of chloroplast [GO:0009507] Sources: GOC:mah